{
  "gene_name": "Protein kinase C and casein kinase substrate in neurons protein 2",
  "term_label": "plasma membrane",
  "gene": "UniProtKB:Q9UNF0",
  "gene_symbol": "PACSIN2",
  "term_id": "GO:0005886"
}